ursodeoxycholate 7-beta-dehydrogenase (NAD+) activity [GO:0106283] (molecular function) Definition: Catalysis of the reaction: NAD+ + ursodeoxycholate = 7-oxolithocholate + H+ + NADH. References: PMID:12917011 Sources: RHEA:42028 Relationships: is a type of GO:0033764